{
  "term_label": "perinuclear region of cytoplasm",
  "term_id": "GO:0048471",
  "gene_symbol": "ALOX12B",
  "gene": "UniProtKB:O75342",
  "gene_name": "Arachidonate 12-lipoxygenase, 12R-type"
}